{
  "term_id": "GO:0005634",
  "gene_symbol": "SERTAD3",
  "gene_name": "SERTA domain-containing protein 3",
  "term_label": "nucleus",
  "gene": "UniProtKB:Q9UJW9"
}